{
  "term_label": "Unknown molecular function",
  "term_id": "UNKNOWN:0001",
  "gene_symbol": "ELOB",
  "gene": "UniProtKB:Q15370",
  "gene_name": "Elongin-B"
}